{
  "term_id": "GO:0140036",
  "gene": "UniProtKB:Q6ZTN6",
  "gene_name": "Ankyrin repeat domain-containing protein 13D",
  "term_label": "ubiquitin-modified protein reader activity",
  "gene_symbol": "ANKRD13D"
}